{
  "term_id": "GO:0005886",
  "gene_symbol": "TRBV11-1",
  "gene": "UniProtKB:A0A0K0K1C0",
  "gene_name": "T cell receptor beta variable 11-1",
  "term_label": "plasma membrane"
}